{
  "term_id": "UNKNOWN:0002",
  "gene_name": "Asparagine synthetase [glutamine-hydrolyzing]",
  "gene_symbol": "ASNS",
  "gene": "UniProtKB:P08243",
  "term_label": "Unknown biological process"
}